ATP transmembrane transporter activity [GO:0005347] (molecular function) Subtypes: GO:0005471, ATP:phosphate antiporter activity [GO:0140987] Relationships: is a type of GO:0000295; is a type of purine ribonucleotide transmembrane transporter activity [GO:0005346]; is part of ATP transport [GO:0015867] Sources: GOC:ai Definition: Enables the transfer of ATP, adenosine triphosphate, from one side of a membrane to the other.